cranial suture morphogenesis [GO:0060363] (biological process) Subtypes: GO:0060364, coronal suture morphogenesis [GO:0060365], GO:0060366, sagittal suture morphogenesis [GO:0060367] Sources: GOC:dph, GOC:pr, GOC:sl Definition: The process in which any suture between cranial bones is generated and organized. Relationships: is a type of GO:0097094